{
  "term_label": "regulation of DNA-templated transcription",
  "gene_name": "Vasculin-like protein 1",
  "term_id": "GO:0006355",
  "gene": "UniProtKB:Q9HC44",
  "gene_symbol": "GPBP1L1"
}